depsipeptide catabolic process [GO:0050762] (biological process) Definition: The chemical reactions and pathways resulting in the breakdown of depsipeptides, a linear or cyclic compound composed of both amino acids and hydroxy acids in peptide and ester bonds respectively. Relationships: is_a catabolic process [GO:0009056]; is a type of GO:0050761 Also known as: depsipeptide breakdown, depsipeptide catabolism, depsipeptide degradation Subtypes: GO:1900556 Sources: GOC:go_curators